positive regulation of secondary metabolite biosynthetic process [GO:1900378] (biological process) Also known as: activation of secondary metabolite biosynthesis, positive regulation of secondary metabolite biosynthesis, up regulation of secondary metabolite biosynthesis, up regulation of secondary metabolite biosynthetic process, up-regulation of secondary metabolite biosynthesis, up-regulation of secondary metabolite biosynthetic process, upregulation of secondary metabolite biosynthesis, upregulation of secondary metabolite biosynthetic process, activation of secondary metabolite biosynthetic process Definition: Any process that activates or increases the frequency, rate or extent of secondary metabolite biosynthetic process. Sources: GOC:TermGenie, GOC:di Subtypes: positive regulation of sterigmatocystin biosynthetic process [GO:0010914], positive regulation of melanin biosynthetic process [GO:0048023], positive regulation of phytoalexin biosynthetic process [GO:0052322], positive regulation terrein biosynthetic process [GO:0140881], GO:1900179, positive regulation of penicillin biosynthetic process [GO:1900198], positive regulation of asperthecin biosynthetic process [GO:1900381], positive regulation of arugosin biosynthetic process [GO:1900628], positive regulation of dehydroaustinol biosynthetic process [GO:1900651], GO:1900654, positive regulation of diorcinol biosynthetic process [GO:1900657], positive regulation of emericellamide biosynthetic process [GO:1900660], positive regulation of emodin biosynthetic process [GO:1900666], positive regulation of endocrocin biosynthetic process [GO:1900669], GO:1900685, positive regulation of gerfelin biosynthetic process [GO:1900688], positive regulation of gliotoxin biosynthetic process [GO:1900691], positive regulation of (+)-kotanin biosynthetic process [GO:1900694], positive regulation of N',N'',N'''-triacetylfusarinine C biosynthetic process [GO:1900697], GO:1900700, positive regulation of orcinol biosynthetic process [GO:1900703], positive regulation of siderophore biosynthetic process [GO:1900706], positive regulation of tensidol A biosynthetic process [GO:1900709], positive regulation of tensidol B biosynthetic process [GO:1900712], positive regulation of violaceol I biosynthetic process [GO:1900715], positive regulation of violaceol II biosynthetic process [GO:1900718], GO:1900734, positive regulation of ergot alkaloid biosynthetic process [GO:1900824], positive regulation of emericellin biosynthetic process [GO:1900836], positive regulation of helvolic acid biosynthetic process [GO:1900842], GO:1900845, positive regulation of terrequinone A biosynthetic process [GO:1900854], positive regulation of cordyol C biosynthetic process [GO:1900863], positive regulation of syringal lignin biosynthetic process [GO:1901430] Relationships: is_a GO:0009891; is a type of regulation of secondary metabolite biosynthetic process [GO:1900376]; positively regulates secondary metabolite biosynthetic process [GO:0044550]